cellular response to granulocyte colony-stimulating factor [GO:1990643] (biological process) Relationships: is a type of cellular response to cytokine stimulus [GO:0071345]; is a type of GO:1990638 Definition: Any process that results in a change in state or activity of a cell (in terms of movement, secretion, enzyme production, gene expression, etc.) as a result of a granulocyte colony-stimulating factor stimulus. References: PMID:9488469